maltotriulose transport [GO:2001090] (BP) Definition: The directed movement of a maltotriuloseacetate into, out of or within a cell, or between cells, by means of some agent such as a transporter or pore. Relationships: is a type of trisaccharide transport [GO:2001088] Sources: GOC:mengo_curators Regulation: regulated by GO:1900324; negatively regulated by negative regulation of maltotriulose transport [GO:1900325]; positively regulated by positive regulation of maltotriulose transport [GO:1900326]